high-affinity tryptophan transmembrane transporter activity [GO:0005300] (molecular function) Definition: Catalysis of the high-affinity transfer of L-tryptophan from one side of a membrane to the other. Tryptophan is 2-amino-3-(1H-indol-3-yl)propanoic acid. In high-affinity transport the transporter is able to bind the solute even if it is only present at very low concentrations. Relationships: is a type of L-tryptophan transmembrane transporter activity [GO:0015196] Sources: GOC:mtg_transport, ISBN:0815340729 Also known as: high-affinity tryptophan transporter activity